{
  "gene_name": "Tubulointerstitial nephritis antigen-like",
  "gene": "UniProtKB:Q9GZM7",
  "term_id": "UNKNOWN:0001",
  "gene_symbol": "TINAGL1",
  "term_label": "Unknown molecular function"
}